{
  "gene_symbol": "TMA7",
  "term_label": "Unknown molecular function",
  "gene_name": "Translation machinery-associated protein 7",
  "term_id": "UNKNOWN:0001",
  "gene": "UniProtKB:Q9Y2S6"
}